{
  "gene_symbol": "ROCK2",
  "gene": "UniProtKB:O75116",
  "term_id": "GO:0048598",
  "gene_name": "Rho-associated protein kinase 2",
  "term_label": "embryonic morphogenesis"
}